{
  "term_label": "RNA endonuclease activity",
  "gene": "UniProtKB:Q9P2P1",
  "term_id": "GO:0004521",
  "gene_symbol": "NYNRIN",
  "gene_name": "Protein NYNRIN"
}